organic acid biosynthetic process [GO:0016053] (biological process) Subtypes: GO:0019295, GO:0019350, alkanesulfonate biosynthetic process [GO:0046305], GO:0046394, teichuronic acid biosynthetic process [GO:0050845] Definition: The chemical reactions and pathways resulting in the formation of organic acids, any acidic compound containing carbon in covalent linkage. Relationships: is a type of organic acid metabolic process [GO:0006082]; is a type of small molecule biosynthetic process [GO:0044283] Sources: ISBN:0198506732 Also known as: organic acid anabolism, organic acid biosynthesis, organic acid formation, organic acid synthesis